{
  "gene_symbol": "SOX30",
  "gene": "UniProtKB:O94993",
  "term_label": "nucleus",
  "term_id": "GO:0005634",
  "gene_name": "Transcription factor SOX-30"
}